{
  "gene_name": "Immunoglobulin heavy variable 3_OR16-12 (non-functional) (Fragment)",
  "gene_symbol": "IGHV3OR16-12",
  "term_id": "UNKNOWN:0003",
  "gene": "UniProtKB:A0A075B7B8",
  "term_label": "Unknown cellular component"
}